ABC-type doxorubicin transporter activity [GO:1901242] (molecular function) Relationships: is a type of GO:0015665; is a type of ABC-type transporter activity [GO:0140359]; is a type of GO:1901505 References: PMID:12057006, PMID:15090538 Sources: GOC:TermGenie Also known as: ATPase-coupled doxorubicin transmembrane transporter activity, doxorubicin transmembrane-transporting ATPase activity Definition: Enables the transfer of a solute or solutes from one side of a membrane to the other according to the reaction: ATP + H2O + doxorubicin(in) = ADP + phosphate + doxorubicin(out).